{
  "gene_symbol": "TMEM8B",
  "gene": "UniProtKB:A6NDV4",
  "term_id": "UNKNOWN:0001",
  "term_label": "Unknown molecular function",
  "gene_name": "Transmembrane protein 8B"
}